{
  "term_label": "transcription cis-regulatory region binding",
  "gene_symbol": "POGZ",
  "gene": "UniProtKB:Q7Z3K3",
  "gene_name": "Pogo transposable element with ZNF domain",
  "term_id": "GO:0000976"
}